talin binding [GO:1990147] (molecular function) Definition: Binding to a talin, a family of related cytoskeletal proteins that play a role in assembly of actin filaments and migration of various cell types. References: PMID:23372168 Sources: GOC:hjd Relationships: is a type of GO:0008092